{
  "gene": "UniProtKB:Q9ULJ8",
  "term_id": "GO:0031175",
  "gene_symbol": "PPP1R9A",
  "term_label": "neuron projection development",
  "gene_name": "Neurabin-1"
}